L-idonate 5-dehydrogenase (NAD+) activity [GO:0102198] (molecular function) Relationships: is a type of L-idonate 5-dehydrogenase [NAD(P)+] activity [GO:0050572] Also known as: L-idonate 5-dehydrogenase activity (NAD-dependent) Definition: Catalysis of the reaction: L-idonate + NAD+ = 5-dehydro-D-gluconate + NADH + H+. Sources: RHEA:21172